{
  "gene": "UniProtKB:Q9Y6X8",
  "gene_symbol": "ZHX2",
  "term_id": "GO:0000981",
  "gene_name": "Zinc fingers and homeoboxes protein 2",
  "term_label": "DNA-binding transcription factor activity, RNA polymerase II-specific"
}